{
  "term_label": "Golgi to vacuole transport",
  "gene_name": "AP-3 complex subunit mu-1",
  "gene_symbol": "AP3M1",
  "gene": "UniProtKB:Q9Y2T2",
  "term_id": "GO:0006896"
}